{
  "term_id": "GO:0035267",
  "term_label": "NuA4 histone acetyltransferase complex",
  "gene": "UniProtKB:Q9NV56",
  "gene_name": "MRG_MORF4L-binding protein",
  "gene_symbol": "MRGBP"
}